ecdysteroid secretion [GO:0045457] (BP) Definition: The regulated release of ecdysteroids, a group of polyhydroxylated ketosteroids which initiate post-embryonic development. Sources: GOC:go_curators Relationships: is a type of steroid hormone secretion [GO:0035929] Regulation: regulated by regulation of ecdysteroid secretion [GO:0007555]; negatively regulated by negative regulation of ecdysteroid secretion [GO:0045999]; RO_0002213 by positive regulation of ecdysteroid secretion [GO:0046000]